{
  "gene_symbol": "KCNK18",
  "term_id": "GO:0015271",
  "gene_name": "Potassium channel subfamily K member 18",
  "term_label": "outward rectifier potassium channel activity",
  "gene": "UniProtKB:Q7Z418"
}